{
  "gene_name": "Heterogeneous nuclear ribonucleoprotein D0",
  "gene_symbol": "HNRNPD",
  "gene": "UniProtKB:Q14103",
  "term_label": "RNA binding",
  "term_id": "GO:0003723"
}